{
  "term_id": "GO:0060287",
  "gene": "UniProtKB:Q9UFE4",
  "term_label": "epithelial cilium movement involved in determination of left/right asymmetry",
  "gene_symbol": "CCDC39",
  "gene_name": "Coiled-coil domain-containing protein 39"
}